{
  "gene_symbol": "ACTG2",
  "term_id": "UNKNOWN:0002",
  "gene_name": "Actin, gamma-enteric smooth muscle",
  "term_label": "Unknown biological process",
  "gene": "UniProtKB:P63267"
}